{
  "gene_symbol": "CHD2",
  "term_label": "nucleus",
  "gene_name": "Chromodomain-helicase-DNA-binding protein 2",
  "term_id": "GO:0005634",
  "gene": "UniProtKB:O14647"
}